{
  "term_label": "plasma membrane",
  "gene_name": "Olfactory receptor 2M4",
  "gene_symbol": "OR2M4",
  "term_id": "GO:0005886",
  "gene": "UniProtKB:Q96R27"
}